regulation of response to salt stress [GO:1901000] (BP) Definition: Any process that modulates the frequency, rate or extent of response to salt stress. Also known as: regulation of response to ionic osmotic stress, regulation of salinity response Relationships: is a type of regulation of response to osmotic stress [GO:0047484]; regulates response to salt stress [GO:0009651] References: PMID:22627139 Sources: GOC:TermGenie Subtypes: regulation of cellular hyperosmotic salinity response [GO:1900069], GO:1901001, positive regulation of response to salt stress [GO:1901002]